{
  "term_id": "GO:0016887",
  "gene": "UniProtKB:Q8NB90",
  "gene_name": "ATPase family gene 2 protein homolog A",
  "term_label": "ATP hydrolysis activity",
  "gene_symbol": "AFG2A"
}